{
  "term_label": "extracellular space",
  "gene_name": "Cysteine-rich secretory protein 1",
  "term_id": "GO:0005615",
  "gene": "UniProtKB:P54107",
  "gene_symbol": "CRISP1"
}